{
  "gene_symbol": "SUMO1",
  "gene_name": "Small ubiquitin-related modifier 1",
  "gene": "UniProtKB:P63165",
  "term_label": "protein sumoylation",
  "term_id": "GO:0016925"
}